peptidyl-pyroglutamic acid biosynthetic process, using glutaminyl-peptide cyclotransferase [GO:0017186] (biological process) Note: See also the molecular function term 'glutaminyl-peptide cyclotransferase activity ; GO:0016603'. Definition: The chemical reactions and pathways resulting in the formation of peptidyl-pyroglutamic acid, catalyzed by glutaminyl-peptide cyclotransferase. Relationships: is a type of GO:0018199 Also known as: 2-pyrrolidone-5-carboxylic acid biosynthesis, 2-pyrrolidone-5-carboxylic acid biosynthetic process, peptidyl-pyroglutamic acid anabolism, using glutaminyl-peptide cyclotransferase, peptidyl-pyroglutamic acid formation, using glutaminyl-peptide cyclotransferase, peptidyl-pyroglutamic acid synthesis, using glutaminyl-peptide cyclotransferase Sources: RESID:AA0031